glucose-1-phospho-D-mannosylglycoprotein phosphodiesterase activity [GO:0047399] (MF) Definition: Catalysis of the reaction: H2O + 6-(D-glucose-1-phospho)-D-mannosylglycoprotein = D-mannosylglycoprotein + D-glucose-alpha-1-phosphate. Relationships: is a type of GO:0008081; is a type of GO:0140103 Also known as: 6-(D-glucose-1-phospho)-D-mannosylglycoprotein glucose-1-phosphohydrolase activity, alpha-glucose-1-phosphate phosphodiesterase activity Sources: EC:3.1.4.51, MetaCyc:3.1.4.51-RXN